nucleoside phosphate metabolic process [GO:0006753] (biological process) Definition: The chemical reactions and pathways involving any phosphorylated nucleoside. Also known as: nucleoside phosphate metabolism Subtypes: GO:0006637, GO:0009117, nucleoside monophosphate metabolic process [GO:0009123], GO:0009132, nucleoside triphosphate metabolic process [GO:0009141], nucleotide-sugar metabolic process [GO:0009225], coenzyme A metabolic process [GO:0015936], nucleoside bisphosphate metabolic process [GO:0033865], nucleoside phosphate catabolic process [GO:1901292], GO:1901293 Relationships: is a type of phosphate-containing compound metabolic process [GO:0006796]; is a type of organophosphate metabolic process [GO:0019637]; is a type of nucleobase-containing small molecule metabolic process [GO:0055086] Sources: GOC:mah